{
  "gene": "UniProtKB:Q8N1C3",
  "gene_name": "Gamma-aminobutyric acid receptor subunit gamma-1",
  "gene_symbol": "GABRG1",
  "term_id": "GO:0004890",
  "term_label": "GABA-A receptor activity"
}